poly(ribitol-phosphate) beta-glucosyltransferase activity [GO:0047266] (molecular function) Definition: Catalysis of the reaction: poly(ribitol phosphate) + UDP-D-glucose = beta-D-glucosylpoly(ribitol phosphate) + UDP. Relationships: is_a UDP-glucosyltransferase activity [GO:0035251] Sources: EC:2.4.1.53 Also known as: UDP glucose-poly(ribitol-phosphate) beta-glucosyltransferase activity, UDP-D-glucose polyribitol phosphate glucosyl transferase activity, UDP-D-glucose:polyribitol phosphate glucosyl transferase activity, UDP-glucose:poly(ribitol-phosphate) beta-D-glucosyltransferase activity, UDPglucose:poly(ribitol-phosphate) beta-D-glucosyltransferase activity, uridine diphosphoglucose-poly(ribitol-phosphate) beta-glucosyltransferase activity